{
  "term_label": "mRNA splicing, via spliceosome",
  "gene": "UniProtKB:P14678",
  "gene_name": "Small nuclear ribonucleoprotein-associated proteins B and B'",
  "gene_symbol": "SNRPB",
  "term_id": "GO:0000398"
}